flavanone 4-reductase activity [GO:0047890] (molecular function) Also known as: flavonone 4-reductase activity, (2S)-flavan-4-ol:NADP+ 4-oxidoreductase activity Definition: Catalysis of the reaction: (2S)-flavan-4-ol + NADP+ = (2S)-flavanone + NADPH. Sources: EC:1.1.1.234, MetaCyc:FLAVANONE-4-REDUCTASE-RXN Relationships: is a type of GO:0016616